{
  "gene": "UniProtKB:Q8WUT9",
  "gene_symbol": "SLC25A43",
  "gene_name": "Solute carrier family 25 member 43",
  "term_label": "Unknown molecular function",
  "term_id": "UNKNOWN:0001"
}